{
  "term_label": "cytoskeleton",
  "gene_symbol": "RAC2",
  "gene": "UniProtKB:P15153",
  "gene_name": "Ras-related C3 botulinum toxin substrate 2",
  "term_id": "GO:0005856"
}